{
  "gene_symbol": "INVS",
  "term_id": "GO:0005929",
  "term_label": "cilium",
  "gene": "UniProtKB:Q9Y283",
  "gene_name": "Inversin"
}